{
  "gene_name": "Integrator complex subunit 14",
  "term_id": "UNKNOWN:0001",
  "gene_symbol": "INTS14",
  "term_label": "Unknown molecular function",
  "gene": "UniProtKB:Q96SY0"
}